{
  "term_label": "troponin I binding",
  "gene": "UniProtKB:P63316",
  "term_id": "GO:0031013",
  "gene_name": "Troponin C, slow skeletal and cardiac muscles",
  "gene_symbol": "TNNC1"
}